{
  "gene_name": "L-lactate dehydrogenase B chain",
  "term_id": "GO:0004459",
  "gene": "UniProtKB:P07195",
  "term_label": "L-lactate dehydrogenase (NAD+) activity",
  "gene_symbol": "LDHB"
}